{
  "gene": "UniProtKB:A6NET4",
  "term_label": "Unknown cellular component",
  "term_id": "UNKNOWN:0003",
  "gene_symbol": "OR5K3",
  "gene_name": "Olfactory receptor 5K3"
}